{
  "term_label": "extracellular matrix",
  "gene": "UniProtKB:Q9NQ76",
  "term_id": "GO:0031012",
  "gene_name": "Matrix extracellular phosphoglycoprotein",
  "gene_symbol": "MEPE"
}